{
  "gene_symbol": "RGS16",
  "term_id": "GO:0045744",
  "term_label": "negative regulation of G protein-coupled receptor signaling pathway",
  "gene_name": "Regulator of G-protein signaling 16",
  "gene": "UniProtKB:O15492"
}